tRNA transcription [GO:0009304] (BP) Definition: The synthesis of transfer RNA (tRNA) from a DNA template. Also known as: tRNA biosynthesis, tRNA biosynthetic process, tRNA synthesis Sources: GOC:jl Relationships: is_a DNA-templated transcription [GO:0006351]; is a type of tRNA metabolic process [GO:0006399] Subtypes: tRNA transcription by RNA polymerase III [GO:0042797]